{
  "gene_name": "Putative gastric cancer-related gene 224 protein",
  "term_label": "Unknown cellular component",
  "gene_symbol": "GCRG224",
  "gene": "UniProtKB:Q8WZA8",
  "term_id": "UNKNOWN:0003"
}